regulation of telium development [GO:0075276] (biological process) Definition: Any process that modulates the frequency, rate or extent of telium development, a process that leads to the formation of a teliospore-bearing sorus of the rust fungi. Subtypes: positive regulation of telium development [GO:0075277], negative regulation of telium development [GO:0075278] Sources: GOC:pamgo_curators Relationships: is a type of regulation of spore-bearing organ development [GO:0075260]; regulates GO:0075275